{
  "gene_name": "Protocadherin beta-13",
  "gene": "UniProtKB:Q9Y5F0",
  "term_id": "GO:0007155",
  "term_label": "cell adhesion",
  "gene_symbol": "PCDHB13"
}